{
  "gene": "UniProtKB:Q9Y224",
  "gene_symbol": "RTRAF",
  "term_label": "tRNA-splicing ligase complex",
  "term_id": "GO:0072669",
  "gene_name": "RNA transcription, translation and transport factor protein"
}